{
  "gene": "UniProtKB:O43236",
  "gene_name": "Septin-4",
  "term_id": "GO:0015630",
  "gene_symbol": "SEPTIN4",
  "term_label": "microtubule cytoskeleton"
}